{
  "gene_symbol": "STRADB",
  "term_label": "protein export from nucleus",
  "gene": "UniProtKB:Q9C0K7",
  "term_id": "GO:0006611",
  "gene_name": "STE20-related kinase adapter protein beta"
}